{
  "gene_symbol": "TMEM97",
  "gene": "UniProtKB:Q5BJF2",
  "gene_name": "Sigma intracellular receptor 2",
  "term_id": "UNKNOWN:0002",
  "term_label": "Unknown biological process"
}